{
  "gene_symbol": "TBL1X",
  "gene": "UniProtKB:O60907",
  "term_label": "histone deacetylase complex",
  "gene_name": "F-box-like_WD repeat-containing protein TBL1X",
  "term_id": "GO:0000118"
}